{
  "term_label": "Unknown molecular function",
  "term_id": "UNKNOWN:0001",
  "gene_name": "Cyclin-D1-binding protein 1",
  "gene_symbol": "CCNDBP1",
  "gene": "UniProtKB:O95273"
}